detection of light stimulus involved in sensory perception [GO:0050962] (biological process) Relationships: is a type of detection of light stimulus [GO:0009583]; is a type of GO:0050906; is part of GO:0050953 Also known as: sensory detection of light stimulus, sensory detection of light stimulus during sensory perception, sensory perception, sensory detection of light stimulus, sensory perception, sensory transduction of light stimulus, sensory transduction of light stimulus, sensory transduction of light stimulus during sensory perception Sources: GOC:ai, GOC:dos Definition: The series of events in which a light stimulus is received by a cell and converted into a molecular signal as part of the sensory perception of light. Subtypes: detection of light stimulus involved in visual perception [GO:0050908], detection of light stimulus involved in magnetoreception [GO:0050980]